pericentric heterochromatin formation [GO:0031508] (biological process) References: PMID:14612388, PMID:20206496, PMID:22729156 Sources: GOC:mah Subtypes: GO:0140727 Relationships: is a type of GO:0140719 Also known as: centromere chromatin silencing, centromeric heterochromatin biosynthesis, centromeric heterochromatin formation, centromeric silencing, chromatin silencing at centromere, heterochromatic silencing at centromere, pericentric heterochromatin assembly, chromatin silencing at centromere outer repeat region, centric heterochromatin formation, chromatin silencing at pericentric region Definition: The compaction of chromatin located adjacent to the CENP-A rich centromere 'central core' and characterized by methylation of histone H3K9, into heterochromatin, resulting in the repression of transcription at pericentric DNA. Regulation: regulated by regulation of pericentric heterochromatin formation [GO:0090052]; positively regulated by GO:0090053